{
  "gene_name": "3 beta-hydroxysteroid dehydrogenase_Delta 5--4-isomerase type 2",
  "term_id": "GO:0005737",
  "term_label": "cytoplasm",
  "gene_symbol": "HSD3B2",
  "gene": "UniProtKB:P26439"
}